{
  "term_id": "GO:0005829",
  "gene": "UniProtKB:Q12882",
  "gene_symbol": "DPYD",
  "term_label": "cytosol",
  "gene_name": "Dihydropyrimidine dehydrogenase [NADP(+)]"
}